{
  "gene_symbol": "ARVCF",
  "term_id": "GO:0098609",
  "term_label": "cell-cell adhesion",
  "gene": "UniProtKB:O00192",
  "gene_name": "Splicing regulator ARVCF"
}